{
  "gene": "UniProtKB:Q5H943",
  "gene_symbol": "CT83",
  "gene_name": "Kita-kyushu lung cancer antigen 1",
  "term_label": "Unknown molecular function",
  "term_id": "UNKNOWN:0001"
}